{
  "term_id": "GO:2000042",
  "gene": "UniProtKB:Q9NWS1",
  "gene_symbol": "PARPBP",
  "gene_name": "PCNA-interacting partner",
  "term_label": "negative regulation of double-strand break repair via homologous recombination"
}